{
  "term_id": "UNKNOWN:0001",
  "gene_name": "Low-density lipoprotein receptor class A domain-containing protein 2",
  "gene": "UniProtKB:Q5SZI1",
  "term_label": "Unknown molecular function",
  "gene_symbol": "LDLRAD2"
}